{
  "gene_symbol": "GNA12",
  "term_id": "GO:0031526",
  "gene": "UniProtKB:Q03113",
  "gene_name": "Guanine nucleotide-binding protein subunit alpha-12",
  "term_label": "brush border membrane"
}